{
  "term_label": "positive regulation of luteinizing hormone secretion",
  "gene_name": "Metastasis-suppressor KiSS-1",
  "term_id": "GO:0033686",
  "gene_symbol": "KISS1",
  "gene": "UniProtKB:Q15726"
}